{
  "term_id": "GO:0005109",
  "gene_name": "Protein Wnt-10a",
  "term_label": "frizzled binding",
  "gene": "UniProtKB:Q9GZT5",
  "gene_symbol": "WNT10A"
}